{
  "gene": "UniProtKB:Q3ZCN5",
  "term_label": "extracellular matrix",
  "gene_name": "Otogelin-like protein",
  "term_id": "GO:0031012",
  "gene_symbol": "OTOGL"
}